{
  "term_id": "GO:0004674",
  "gene_name": "Mitogen-activated protein kinase kinase kinase 12",
  "term_label": "protein serine/threonine kinase activity",
  "gene_symbol": "MAP3K12",
  "gene": "UniProtKB:Q12852"
}